{
  "term_id": "GO:0005783",
  "gene_symbol": "HHATL",
  "term_label": "endoplasmic reticulum",
  "gene": "UniProtKB:Q9HCP6",
  "gene_name": "Protein-cysteine N-palmitoyltransferase HHAT-like protein"
}